{
  "term_id": "GO:0070679",
  "gene_symbol": "TRPC6",
  "gene": "UniProtKB:Q9Y210",
  "term_label": "inositol 1,4,5 trisphosphate binding",
  "gene_name": "Short transient receptor potential channel 6"
}